positive aerotaxis [GO:0052131] (biological process) Relationships: is a type of aerotaxis [GO:0009454]; is a type of GO:0050918; is a type of positive energy taxis [GO:0052128] Sources: GOC:dph, GOC:mtg_pamgo_17jul06 Definition: The directed movement of a motile cell or organism towards a higher concentration of environmental oxygen.